pantetheine hydrolase activity [GO:0017159] (molecular function) Also known as: (R)-pantetheine amidohydrolase activity, pantetheinase activity, vanin, vanin-1 Definition: Catalysis of the reaction: (R)-pantetheine + H2O = (R)-pantothenate + cysteamine. Relationships: is a type of hydrolase activity, acting on carbon-nitrogen (but not peptide) bonds, in linear amides [GO:0016811] Sources: EC:3.5.1.92, RHEA:13445